{
  "gene_symbol": "S100Z",
  "term_id": "UNKNOWN:0002",
  "term_label": "Unknown biological process",
  "gene": "UniProtKB:Q8WXG8",
  "gene_name": "Protein S100-Z"
}